negative regulation of transforming growth factor beta1 production [GO:0032911] (biological process) Relationships: is a type of regulation of transforming growth factor beta1 production [GO:0032908]; is a type of negative regulation of transforming growth factor beta production [GO:0071635]; negatively regulates transforming growth factor beta1 production [GO:0032905] Sources: GOC:mah Also known as: down regulation of transforming growth factor-beta1 production, down-regulation of transforming growth factor-beta1 production, downregulation of transforming growth factor-beta1 production, negative regulation of TGF-B1 production, negative regulation of TGFB1 production, negative regulation of transforming growth factor-beta1 production, inhibition of transforming growth factor-beta1 production Definition: Any process that stops, prevents, or reduces the frequency, rate, or extent of production of transforming growth factor-beta1.